{
  "term_label": "Unknown biological process",
  "gene": "UniProtKB:Q96PY0",
  "gene_symbol": "PSMG3-AS1",
  "gene_name": "Putative uncharacterized protein PSMG3-AS1",
  "term_id": "UNKNOWN:0002"
}